G protein-coupled ADP receptor activity [GO:0001621] (molecular function) Relationships: is a type of G protein-coupled purinergic nucleotide receptor activity [GO:0045028]; BFO_0000051 ADP binding [GO:0043531] Also known as: ADP receptor activity, ADP-activated nucleotide receptor activity, K101 receptor, platelet ADP receptor activity, ADP-activated adenosine receptor activity References: PMID:11196645 Sources: GOC:mah, GOC:signaling Definition: Combining with ADP and transmitting the signal across the membrane by activating an associated G-protein; promotes the exchange of GDP for GTP on the alpha subunit of a heterotrimeric G-protein complex.